{
  "gene_symbol": "FGG",
  "term_id": "GO:0007160",
  "term_label": "cell-matrix adhesion",
  "gene": "UniProtKB:P02679",
  "gene_name": "Fibrinogen gamma chain"
}